{
  "gene_name": "Kv channel-interacting protein 1",
  "gene": "UniProtKB:Q9NZI2",
  "term_label": "calcium ion binding",
  "gene_symbol": "KCNIP1",
  "term_id": "GO:0005509"
}